{
  "gene_name": "Syntaxin-binding protein 5-like",
  "gene_symbol": "STXBP5L",
  "gene": "UniProtKB:Q9Y2K9",
  "term_id": "GO:0005096",
  "term_label": "GTPase activator activity"
}